reelin-mediated signaling pathway [GO:0038026] (biological process) Also known as: reeler-mediated signaling pathway, reelin-mediated signal transduction pathway, reelin-mediated signalling pathway Definition: The series of molecular signals initiated by the binding of reelin (a secreted glycoprotein) to a receptor on the surface of a target cell, and ending with the regulation of a downstream cellular process, e.g. transcription. Relationships: is a type of cell surface receptor signaling pathway [GO:0007166] References: PMID:12827279, PMID:20223215 Sources: GOC:bf